{
  "term_id": "GO:0005634",
  "gene_name": "Fos-related antigen 2",
  "gene": "UniProtKB:P15408",
  "gene_symbol": "FOSL2",
  "term_label": "nucleus"
}